{
  "gene_symbol": "CLDN11",
  "gene": "UniProtKB:O75508",
  "term_label": "tight junction assembly",
  "term_id": "GO:0120192",
  "gene_name": "Claudin-11"
}